{
  "term_id": "GO:0005634",
  "gene": "UniProtKB:Q9P0W2",
  "gene_name": "SWI_SNF-related matrix-associated actin-dependent regulator of chromatin subfamily E member 1-related",
  "term_label": "nucleus",
  "gene_symbol": "HMG20B"
}